{
  "term_id": "GO:0004802",
  "term_label": "transketolase activity",
  "gene_symbol": "TKT",
  "gene_name": "Transketolase",
  "gene": "UniProtKB:P29401"
}